{
  "term_id": "UNKNOWN:0003",
  "gene_symbol": "HDX",
  "term_label": "Unknown cellular component",
  "gene": "UniProtKB:Q7Z353",
  "gene_name": "Highly divergent homeobox"
}